{
  "gene_name": "Selenocysteine insertion sequence-binding protein 2-like",
  "gene": "UniProtKB:Q93073",
  "term_label": "ribonucleoprotein complex binding",
  "gene_symbol": "SECISBP2L",
  "term_id": "GO:0043021"
}